{
  "term_label": "nicotinate-nucleotide diphosphorylase (carboxylating) activity",
  "gene_name": "Nicotinate-nucleotide pyrophosphorylase [carboxylating]",
  "term_id": "GO:0004514",
  "gene_symbol": "QPRT",
  "gene": "UniProtKB:Q15274"
}